{
  "term_label": "regulation of mitochondrial membrane permeability",
  "gene_name": "ADP_ATP translocase 3",
  "term_id": "GO:0046902",
  "gene_symbol": "SLC25A6",
  "gene": "UniProtKB:P12236"
}